(S)-corytuberine synthase activity [GO:0102963] (molecular function) Definition: Catalysis of the reaction: H+ + (S)-reticulinium(1+) + NADPH + O2 = (S)-corytuberine + NADP + 2 H2O. References: PMID:18230623 Sources: RHEA:51540 Relationships: is a type of oxidoreductase activity, acting on paired donors, with oxidation of a pair of donors resulting in the reduction of molecular oxygen to two molecules of water [GO:0016717]